positive regulation of serine C-palmitoyltransferase activity [GO:1904222] (biological process) References: PMID:16120614 Sources: GOC:BHF, GOC:TermGenie, GOC:rl, GO_REF:0000059 Definition: Any process that activates or increases the frequency, rate or extent of serine C-palmitoyltransferase activity. Relationships: is a type of positive regulation of catalytic activity [GO:0043085]; is a type of regulation of transferase activity [GO:0051338]; positively regulates serine C-palmitoyltransferase activity [GO:0004758] Note: Serinc proteins form a complex with serine and sphingolipid biosynthesis enzymes and regulates their activity through regulation of the substrate availability Also known as: positive regulation of 3-oxosphinganine synthetase activity, positive regulation of palmitoyl-CoA:L-serine C-palmitoyltransferase (decarboxylating) activity, up regulation of 3-oxosphinganine synthetase activity, up regulation of palmitoyl-CoA:L-serine C-palmitoyltransferase (decarboxylating) activity, up regulation of serine C-palmitoyltransferase activity, up-regulation of 3-oxosphinganine synthetase activity, up-regulation of palmitoyl-CoA:L-serine C-palmitoyltransferase (decarboxylating) activity, up-regulation of serine C-palmitoyltransferase activity, upregulation of 3-oxosphinganine synthetase activity, upregulation of palmitoyl-CoA:L-serine C-palmitoyltransferase (decarboxylating) activity, upregulation of serine C-palmitoyltransferase activity, activation of 3-oxosphinganine synthetase activity, activation of palmitoyl-CoA:L-serine C-palmitoyltransferase (decarboxylating) activity, activation of serine C-palmitoyltransferase activity, activation of SPT, activation of acyl-CoA:serine C-2 acyltransferase decarboxylating, positive regulation of SPT, positive regulation of acyl-CoA:serine C-2 acyltransferase decarboxylating, up regulation of SPT, up regulation of acyl-CoA:serine C-2 acyltransferase decarboxylating, up-regulation of SPT, up-regulation of acyl-CoA:serine C-2 acyltransferase decarboxylating, upregulation of SPT, upregulation of acyl-CoA:serine C-2 acyltransferase decarboxylating